{
  "gene_name": "Translation machinery-associated protein 16",
  "gene_symbol": "TMA16",
  "gene": "UniProtKB:Q96EY4",
  "term_label": "Unknown biological process",
  "term_id": "UNKNOWN:0002"
}